Rho GDP-dissociation inhibitor binding [GO:0051022] (molecular function) Definition: Binding to a Rho GDP-dissociation inhibitor protein. Relationships: is a type of GDP-dissociation inhibitor binding [GO:0051021] Sources: GOC:ai Also known as: Rho GDI binding